{
  "term_label": "actin-based cell projection",
  "gene": "UniProtKB:Q9P2A4",
  "gene_name": "ABI gene family member 3",
  "gene_symbol": "ABI3",
  "term_id": "GO:0098858"
}